{
  "term_id": "GO:0009612",
  "term_label": "response to mechanical stimulus",
  "gene": "UniProtKB:P45983",
  "gene_symbol": "MAPK8",
  "gene_name": "Mitogen-activated protein kinase 8"
}